{
  "term_id": "GO:0016477",
  "gene": "UniProtKB:Q9Y5K6",
  "term_label": "cell migration",
  "gene_symbol": "CD2AP",
  "gene_name": "CD2-associated protein"
}